blood vessel remodeling [GO:0001974] (biological process) Also known as: blood vessel remodelling Definition: The reorganization or renovation of existing blood vessels. Sources: GOC:hjd Regulation: regulated by regulation of blood vessel remodeling [GO:0060312]; RO_0002212 by negative regulation of blood vessel remodeling [GO:0060313]; positively regulated by positive regulation of blood vessel remodeling [GO:2000504] Relationships: is a type of tissue remodeling [GO:0048771] Subtypes: pulmonary blood vessel remodeling [GO:0101010]